{
  "gene": "UniProtKB:Q15836",
  "term_label": "plasma membrane",
  "gene_symbol": "VAMP3",
  "term_id": "GO:0005886",
  "gene_name": "Vesicle-associated membrane protein 3"
}